{
  "gene_symbol": "RBFOX3",
  "gene_name": "RNA binding protein fox-1 homolog 3",
  "term_id": "GO:0007399",
  "term_label": "nervous system development",
  "gene": "UniProtKB:A6NFN3"
}